{
  "term_label": "cytosol",
  "gene": "UniProtKB:P82980",
  "gene_symbol": "RBP5",
  "term_id": "GO:0005829",
  "gene_name": "Retinol-binding protein 5"
}